{
  "gene_name": "Cytokine receptor-like factor 1",
  "term_id": "GO:0097058",
  "gene": "UniProtKB:O75462",
  "gene_symbol": "CRLF1",
  "term_label": "CRLF-CLCF1 complex"
}